{
  "gene": "UniProtKB:Q8NFP7",
  "term_id": "GO:0000298",
  "gene_name": "Diphosphoinositol polyphosphate phosphohydrolase 3-alpha",
  "term_label": "endopolyphosphatase activity",
  "gene_symbol": "NUDT10"
}